regulation of direction of cell growth [GO:0061389] (BP) Sources: GOC:mah, GOC:vw Definition: Any process that modulates the direction of cell growth. Relationships: is a type of regulation of cell growth [GO:0001558]; is a type of regulation of cell shape [GO:0008360] Subtypes: cell growth mode switching, monopolar to bipolar [GO:0051523], cell growth mode switching, bipolar to monopolar [GO:0051524], positive regulation of direction of cell growth [GO:0061390], negative regulation of direction of cell growth [GO:0061391]